{
  "gene_name": "Zinc finger protein 74",
  "gene": "UniProtKB:Q16587",
  "gene_symbol": "ZNF74",
  "term_label": "regulation of transcription by RNA polymerase II",
  "term_id": "GO:0006357"
}